negative regulation of catecholamine uptake involved in synaptic transmission [GO:0051945] (biological process) Relationships: is a type of negative regulation of neurotransmitter uptake [GO:0051581]; is a type of GO:0051940; is a type of negative regulation of amine transport [GO:0051953]; negatively regulates catecholamine uptake involved in synaptic transmission [GO:0051934] Sources: GOC:ai, GOC:dph, GOC:tb Definition: Any process that stops, prevents, or reduces the frequency, rate or extent of the directed movement of catecholamine neurotransmitters into a neuron or glial cell. Subtypes: negative regulation of dopamine uptake involved in synaptic transmission [GO:0051585] Also known as: negative regulation of catecholamine uptake during transmission of nerve impulse, down regulation of catecholamine uptake during transmission of nerve impulse, down-regulation of catecholamine uptake during transmission of nerve impulse, downregulation of catecholamine uptake during transmission of nerve impulse, negative regulation of catecholamine neurotransmitter reuptake, negative regulation of catecholamine neurotransmitter uptake, inhibition of catecholamine uptake during transmission of nerve impulse